{
  "gene_name": "Neuronal tyrosine-phosphorylated phosphoinositide-3-kinase adapter 2",
  "gene_symbol": "NYAP2",
  "gene": "UniProtKB:Q9P242",
  "term_id": "UNKNOWN:0001",
  "term_label": "Unknown molecular function"
}